platelet activating factor catabolic process [GO:0062234] (biological process) Definition: The chemical reactions and pathways resulting in the breakdown of platelet activating factor, 2-O-acetyl-1-O-octadecyl-sn-glycero-3-phosphocholine. References: PMID:16371369 Also known as: 2-O-acetyl-1-O-octadecyl-sn-glycero-3-phosphocholine catabolic process, PAF catabolic process Relationships: is_a glycerol ether catabolic process [GO:0044269]; is a type of platelet activating factor metabolic process [GO:0046469]; is a type of glycerophospholipid catabolic process [GO:0046475]